{
  "term_id": "GO:0048487",
  "gene_symbol": "TBCD",
  "gene": "UniProtKB:Q9BTW9",
  "gene_name": "Tubulin-specific chaperone D",
  "term_label": "beta-tubulin binding"
}